negative regulation of NLRP3 inflammasome complex assembly [GO:1900226] (biological process) Definition: Any process that stops, prevents or reduces the frequency, rate or extent of NLRP3 inflammasome complex assembly. Also known as: down regulation of NALP3 inflammasome complex assembly, down regulation of NLRP3 inflammasome complex assembly, down-regulation of NALP3 inflammasome complex assembly, down-regulation of NLRP3 inflammasome complex assembly, downregulation of NALP3 inflammasome complex assembly, downregulation of NLRP3 inflammasome complex assembly, inhibition of NALP3 inflammasome complex assembly, negative regulation of NALP3 inflammasome complex assembly, inhibition of NLRP3 inflammasome complex assembly, down regulation of NLRP3 inflammasome activation, down-regulation of NLRP3 inflammasome activation, downregulation of NLRP3 inflammasome activation, inhibition of NLRP3 inflammasome activation, negative regulation of NLRP3 inflammasome activation Sources: GOC:TermGenie Relationships: is a type of negative regulation of protein-containing complex assembly [GO:0031333]; is a type of regulation of NLRP3 inflammasome complex assembly [GO:1900225]; is part of negative regulation of inflammasome-mediated signaling pathway [GO:0141086]; negatively regulates NLRP3 inflammasome complex assembly [GO:0044546]